short-chain fatty acid catabolic process [GO:0019626] (biological process) Sources: ISBN:0198506732 Definition: The chemical reactions and pathways resulting in the breakdown of a short-chain fatty acid. A short-chain fatty acid has an aliphatic tail containing fewer than 6 carbons. Note: While there is not universal consensus on the lengths of short-, medium-, long- and very-long-chain fatty acids, the GO uses the definitions in ChEBI (see CHEBI:26666, CHEBI:59554, CHEBI:15904 and CHEBI:27283). Also known as: short-chain fatty acid breakdown, short-chain fatty acid catabolism, short-chain fatty acid degradation Subtypes: propionate catabolic process [GO:0019543], 2-oxobutyrate catabolic process [GO:0019606], acetoacetic acid catabolic process [GO:0043442], butyrate catabolic process [GO:0046359] Relationships: is a type of fatty acid catabolic process [GO:0009062]; is a type of GO:0046459